{
  "gene": "UniProtKB:Q3SY77",
  "gene_symbol": "UGT3A2",
  "term_label": "UDP-N-acetylglucosamine transferase complex",
  "gene_name": "UDP-glucuronosyltransferase 3A2",
  "term_id": "GO:0043541"
}